{
  "gene_symbol": "CA5A",
  "term_label": "mitochondrion",
  "gene_name": "Carbonic anhydrase 5A, mitochondrial",
  "gene": "UniProtKB:P35218",
  "term_id": "GO:0005739"
}